{
  "gene_symbol": "TBX3",
  "gene_name": "T-box transcription factor TBX3",
  "term_label": "regulation of transcription by RNA polymerase II",
  "term_id": "GO:0006357",
  "gene": "UniProtKB:O15119"
}